{
  "term_label": "microtubule",
  "gene": "UniProtKB:Q2M1P5",
  "term_id": "GO:0005874",
  "gene_name": "Kinesin-like protein KIF7",
  "gene_symbol": "KIF7"
}